regulation of alpha-glucan metabolic process [GO:0032948] (biological process) Relationships: is a type of regulation of polysaccharide metabolic process [GO:0032881]; regulates alpha-glucan metabolic process [GO:0030978] Sources: GOC:mah Subtypes: GO:0032949 Definition: Any process that modulates the frequency, rate or extent of the chemical reactions and pathways involving alpha-glucans. Also known as: regulation of alpha-glucan metabolism